{
  "gene": "UniProtKB:Q99567",
  "gene_name": "Nuclear pore complex protein Nup88",
  "term_id": "GO:0006406",
  "gene_symbol": "NUP88",
  "term_label": "mRNA export from nucleus"
}